{
  "term_label": "CCR6 chemokine receptor binding",
  "gene_name": "Beta-defensin 110",
  "gene_symbol": "DEFB110",
  "term_id": "GO:0031731",
  "gene": "UniProtKB:Q30KQ9"
}